fatty acid elongation, unsaturated fatty acid [GO:0019368] (biological process) Definition: Elongation of a fatty acid chain into which one or more C-C double bonds have been introduced. Relationships: is a type of fatty acid elongation [GO:0030497] Subtypes: fatty acid elongation, monounsaturated fatty acid [GO:0034625], fatty acid elongation, polyunsaturated fatty acid [GO:0034626] Sources: GOC:mah